{
  "term_label": "Unknown molecular function",
  "gene": "UniProtKB:H3BQL2",
  "term_id": "UNKNOWN:0001",
  "gene_name": "Golgin subfamily A member 8T",
  "gene_symbol": "GOLGA8T"
}